tertiary granule membrane [GO:0070821] (cellular component) References: PMID:12070036 Sources: GOC:BHF, GOC:mah, GOC:rl Relationships: is a type of secretory granule membrane [GO:0030667]; is part of GO:0070820 Definition: The lipid bilayer surrounding a tertiary granule.